{
  "gene_symbol": "SLN",
  "gene_name": "Sarcolipin",
  "term_id": "GO:0016529",
  "term_label": "sarcoplasmic reticulum",
  "gene": "UniProtKB:O00631"
}